{
  "gene": "UniProtKB:Q16873",
  "gene_symbol": "LTC4S",
  "term_label": "leukotriene-C4 synthase activity",
  "term_id": "GO:0004464",
  "gene_name": "Leukotriene C4 synthase"
}